vitamin E biosynthetic process [GO:0010189] (biological process) Regulation: regulated by regulation of vitamin E biosynthetic process [GO:1904965]; positively regulated by positive regulation of vitamin E biosynthetic process [GO:1904966] Sources: GOC:mg Definition: The chemical reactions and pathways resulting in the formation of vitamin E, tocopherol, which includes a series of eight structurally similar compounds. Alpha-tocopherol is the most active form in humans and is a powerful biological antioxidant. Relationships: is a type of GO:0042360; is a type of fat-soluble vitamin biosynthetic process [GO:0042362] Also known as: tocopherol biosynthesis, tocopherol biosynthetic process, vitamin E anabolism, vitamin E biosynthesis, vitamin E formation, vitamin E synthesis, alpha-tocopherol biosynthesis, alpha-tocopherol biosynthetic process